{
  "gene_symbol": "SCO2",
  "term_id": "GO:0033617",
  "gene": "UniProtKB:O43819",
  "gene_name": "Protein SCO2 homolog, mitochondrial",
  "term_label": "mitochondrial respiratory chain complex IV assembly"
}